{
  "term_label": "ferrous iron binding",
  "gene_symbol": "ALKBH1",
  "gene_name": "Nucleic acid dioxygenase ALKBH1",
  "term_id": "GO:0008198",
  "gene": "UniProtKB:Q13686"
}